{
  "gene_symbol": "IFNL2",
  "term_id": "GO:0051607",
  "gene_name": "Interferon lambda-2",
  "gene": "UniProtKB:Q8IZJ0",
  "term_label": "defense response to virus"
}